(+)-3'-hydroxylarreatricin biosynthetic process [GO:1901708] (biological process) References: PMID:12960376 Sources: GOC:TermGenie Also known as: (+)-3'-hydroxylarreatricin anabolism, (+)-3'-hydroxylarreatricin biosynthesis, (+)-3'-hydroxylarreatricin formation, (+)-3'-hydroxylarreatricin synthesis Relationships: is a type of lignan biosynthetic process [GO:0009807] Definition: The chemical reactions and pathways resulting in the formation of (+)-3'-hydroxylarreatricin.